negative regulation of neurotrophin TRK receptor signaling pathway [GO:0051387] (biological process) Also known as: down regulation of nerve growth factor receptor signaling pathway, down-regulation of nerve growth factor receptor signaling pathway, downregulation of nerve growth factor receptor signaling pathway, negative regulation of NGF receptor signaling pathway, negative regulation of NGF receptor signalling pathway, negative regulation of nerve growth factor receptor signalling pathway, inhibition of nerve growth factor receptor signaling pathway, negative regulation of nerve growth factor receptor signaling pathway Relationships: is a type of negative regulation of signal transduction [GO:0009968]; is a type of regulation of neurotrophin TRK receptor signaling pathway [GO:0051386]; is a type of negative regulation of cellular response to growth factor stimulus [GO:0090288]; negatively regulates neurotrophin TRK receptor signaling pathway [GO:0048011] Definition: Any process that stops, prevents, or reduces the frequency, rate or extent of the neurotrophin TRK receptor signaling pathway. Sources: GOC:ai